{
  "gene_name": "Replication factor C subunit 5",
  "gene": "UniProtKB:P40937",
  "term_id": "GO:0006261",
  "term_label": "DNA-templated DNA replication",
  "gene_symbol": "RFC5"
}